regulation of gastric mucosal blood circulation [GO:1904344] (biological process) Also known as: regulation of stomach mucosal blood circulation Relationships: is a type of regulation of blood circulation [GO:1903522]; regulates gastric mucosal blood circulation [GO:1990768] References: PMID:10807413 Sources: GOC:TermGenie, GO_REF:0000058 Definition: Any process that modulates the frequency, rate or extent of gastric mucosal blood circulation. Subtypes: negative regulation of gastric mucosal blood circulation [GO:1904345], positive regulation of gastric mucosal blood circulation [GO:1904346]